telomerase RNA localization to Cajal body [GO:0090671] (biological process) Definition: A process in which telomerase RNA (TERC) is transported to, or maintained in, a Cajal body. References: PMID:25467444 Sources: GOC:BHF, GOC:BHF_telomere, GOC:nc Relationships: is a type of RNA localization to Cajal body [GO:0090670]; is a type of telomerase RNA localization [GO:0090672] Regulation: regulated by regulation of telomerase RNA localization to Cajal body [GO:1904872]; negatively regulated by negative regulation of telomerase RNA localization to Cajal body [GO:1904873]; positively regulated by positive regulation of telomerase RNA localization to Cajal body [GO:1904874]